{
  "term_label": "Unknown cellular component",
  "term_id": "UNKNOWN:0003",
  "gene_name": "Putative uncharacterized protein DKFZp434L187",
  "gene_symbol": "Q9UFV3",
  "gene": "UniProtKB:Q9UFV3"
}